{
  "gene_symbol": "PRR5L",
  "gene": "UniProtKB:Q6MZQ0",
  "term_label": "TORC2 signaling",
  "term_id": "GO:0038203",
  "gene_name": "Proline-rich protein 5-like"
}